thylakoid membrane [GO:0042651] (CC) Subtypes: plasma membrane-derived thylakoid membrane [GO:0031676], plastid thylakoid membrane [GO:0055035], organellar chromatophore thylakoid membrane [GO:0070118] Definition: The pigmented membrane of any thylakoid. Relationships: is a type of photosynthetic membrane [GO:0034357] Sources: GOC:jl, GOC:pr